CLRC complex [GO:0043494] (cellular component) Relationships: is a type of nuclear ubiquitin ligase complex [GO:0000152]; is a type of GO:0035097; is a type of Cul4-RING E3 ubiquitin ligase complex [GO:0080008] Also known as: CLRC ubiquitin ligase complex, Clr4-Rik1-Cul4 complex, Rik1 E3 ubiquitin ligase complex, Rik1-E3 ubiquitin ligase complex References: PMID:16127433, PMID:20211136 Sources: GOC:vw Definition: An cullin-dependent E3 ubiquitin ligase/histone H3-K9 methyltransferase complex essential for heterochromatin assembly by RNAi.